sexual reproduction [GO:0019953] (BP) Definition: A type of reproduction that combines the genetic material of two gametes (such as a sperm or egg cell or fungal spores). The gametes have an haploid genome (with a single set of chromosomes, the product of a meiotic division) and combines with one another to produce a zygote (diploid). Sources: Wikipedia:Sexual_reproduction Relationships: is a type of reproductive process [GO:0022414] Subtypes: GO:0000747, GO:0000748 Note: Note that gametes may come from two organisms or from a single organism in the case of self-fertilizing hermaphrodites, e.g. C. elegans, or self-fertilization in plants. Note also that sexual reproduction may be seen as the regular alternation, in the life cycle of haplontic, diplontic and diplohaplontic organisms, of meiosis and fertilization which provides for the production offspring. In diplontic organisms there is a life cycle in which the products of meiosis behave directly as gametes, fusing to form a zygote from which the diploid, or sexually reproductive polyploid, adult organism will develop. In diplohaplontic organisms a haploid phase (gametophyte) exists in the life cycle between meiosis and fertilization (e.g. higher plants, many algae and Fungi); the products of meiosis are spores that develop as haploid individuals from which haploid gametes develop to form a diploid zygote; diplohaplontic organisms show an alternation of haploid and diploid generations. In haplontic organisms meiosis occurs in the zygote, giving rise to four haploid cells (e.g. many algae and protozoa), only the zygote is diploid and this may form a resistant spore, tiding organisms over hard times.